{
  "gene": "UniProtKB:Q9P0J7",
  "term_label": "synaptic signaling",
  "term_id": "GO:0099536",
  "gene_symbol": "KCMF1",
  "gene_name": "E3 ubiquitin-protein ligase KCMF1"
}